{
  "term_id": "UNKNOWN:0001",
  "term_label": "Unknown molecular function",
  "gene_name": "Brevican core protein",
  "gene": "UniProtKB:Q96GW7",
  "gene_symbol": "BCAN"
}